{
  "term_label": "positive regulation of Wnt signaling pathway",
  "gene_symbol": "SULF1",
  "gene": "UniProtKB:Q8IWU6",
  "gene_name": "Extracellular sulfatase Sulf-1",
  "term_id": "GO:0030177"
}